{
  "gene": "UniProtKB:O00470",
  "term_label": "nucleus",
  "gene_name": "Homeobox protein Meis1",
  "gene_symbol": "MEIS1",
  "term_id": "GO:0005634"
}